{
  "term_id": "GO:0002009",
  "gene_name": "Keratin, type I cuticular Ha2",
  "gene_symbol": "KRT32",
  "term_label": "morphogenesis of an epithelium",
  "gene": "UniProtKB:Q14532"
}